{
  "gene": "UniProtKB:Q5VZR2",
  "gene_name": "NUT family member 2G",
  "term_id": "UNKNOWN:0002",
  "term_label": "Unknown biological process",
  "gene_symbol": "NUTM2G"
}